positive regulation of L-dopa biosynthetic process [GO:1903197] (biological process) Also known as: positive regulation of L-dopa anabolism, positive regulation of L-dopa biosynthesis, positive regulation of L-dopa formation, positive regulation of L-dopa synthesis, up regulation of L-dopa anabolism, up regulation of L-dopa biosynthesis, up regulation of L-dopa biosynthetic process, up regulation of L-dopa formation, up regulation of L-dopa synthesis, up-regulation of L-dopa anabolism, up-regulation of L-dopa biosynthesis, up-regulation of L-dopa biosynthetic process, up-regulation of L-dopa formation, up-regulation of L-dopa synthesis, upregulation of L-dopa anabolism, upregulation of L-dopa biosynthesis, upregulation of L-dopa biosynthetic process, upregulation of L-dopa formation, upregulation of L-dopa synthesis, activation of L-dopa anabolism, activation of L-dopa biosynthesis, activation of L-dopa biosynthetic process, activation of L-dopa formation, activation of L-dopa synthesis Relationships: is a type of positive regulation of small molecule metabolic process [GO:0062013]; is a type of regulation of L-dopa biosynthetic process [GO:1903195]; is a type of GO:2000284; positively regulates L-dopa biosynthetic process [GO:1903185] References: PMID:16731528 Sources: GOC:PARL, GOC:TermGenie, GOC:bf, GO_REF:0000058 Definition: Any process that activates or increases the frequency, rate or extent of L-dopa biosynthetic process.